{
  "gene_symbol": "NUP210L",
  "gene_name": "Nuclear pore membrane glycoprotein 210-like",
  "term_label": "Unknown molecular function",
  "term_id": "UNKNOWN:0001",
  "gene": "UniProtKB:Q5VU65"
}